{
  "gene_name": "X-linked retinitis pigmentosa GTPase regulator",
  "gene": "UniProtKB:Q92834",
  "term_id": "GO:0005794",
  "gene_symbol": "RPGR",
  "term_label": "Golgi apparatus"
}